{
  "gene_name": "TATA-box-binding protein-associated factor 11-like protein 4",
  "term_label": "RNA polymerase II preinitiation complex assembly",
  "term_id": "GO:0051123",
  "gene": "UniProtKB:A0A1W2PPE2",
  "gene_symbol": "TAF11L4"
}